{
  "gene_name": "Doublecortin domain-containing protein 2",
  "gene": "UniProtKB:Q9UHG0",
  "term_id": "UNKNOWN:0001",
  "term_label": "Unknown molecular function",
  "gene_symbol": "DCDC2"
}